equilibrioception [GO:0050957] (biological process) Relationships: is a type of sensory perception [GO:0007600]; is part of neuromuscular process controlling balance [GO:0050885] Definition: The series of events required for an organism to receive an orientational stimulus, convert it to a molecular signal, and recognize and characterize the signal. Equilibrioception refers to a combination of processes by which an organism can perceive its orientation with respect to gravity. In animals, stimuli come from labyrinth system of the inner ears, monitoring the direction of motion; visual stimuli, with information on orientation and motion; pressure receptors, which tell the organism which body surfaces are in contact with the ground; and proprioceptive cues, which report which parts of the body are in motion. Also known as: sensory perception of orientation with respect to gravity References: PMID:29303967